{
  "gene_symbol": "FEN1",
  "term_id": "UNKNOWN:0002",
  "gene_name": "Flap endonuclease 1",
  "term_label": "Unknown biological process",
  "gene": "UniProtKB:P39748"
}